{
  "gene": "UniProtKB:Q9Y6C7",
  "gene_name": "Putative uncharacterized protein encoded by LINC00312",
  "term_label": "Unknown cellular component",
  "gene_symbol": "LINC00312",
  "term_id": "UNKNOWN:0003"
}